{
  "gene_symbol": "RAB5A",
  "term_label": "GTPase activity",
  "gene_name": "Ras-related protein Rab-5A",
  "gene": "UniProtKB:P20339",
  "term_id": "GO:0003924"
}